{
  "term_id": "GO:0005604",
  "gene": "UniProtKB:Q63HQ2",
  "gene_name": "Pikachurin",
  "term_label": "basement membrane",
  "gene_symbol": "EGFLAM"
}